gallate decarboxylase activity [GO:0018798] (molecular function) Definition: Catalysis of the reaction: gallate + H+ = CO2 + pyrogallol. Also known as: gallic acid decarboxylase activity, gallate carboxy-lyase (pyrogallol-forming), gallate carboxy-lyase activity Relationships: is_a carboxy-lyase activity [GO:0016831] Sources: EC:4.1.1.59, RHEA:12749